{
  "term_id": "GO:0044323",
  "gene": "UniProtKB:P28702",
  "term_label": "retinoic acid-responsive element binding",
  "gene_name": "Retinoic acid receptor RXR-beta",
  "gene_symbol": "RXRB"
}